{
  "term_id": "GO:1990130",
  "gene_symbol": "NPRL2",
  "gene_name": "GATOR complex protein NPRL2",
  "term_label": "GATOR1 complex",
  "gene": "UniProtKB:Q8WTW4"
}